{
  "gene_name": "BolA-like protein 2",
  "term_id": "GO:0051536",
  "gene_symbol": "BOLA2",
  "term_label": "iron-sulfur cluster binding",
  "gene": "UniProtKB:Q9H3K6"
}